{
  "gene_symbol": "ARID1A",
  "term_id": "GO:0071565",
  "gene_name": "AT-rich interactive domain-containing protein 1A",
  "term_label": "nBAF complex",
  "gene": "UniProtKB:O14497"
}